{
  "term_id": "GO:0007099",
  "gene": "UniProtKB:Q6UVJ0",
  "gene_name": "Spindle assembly abnormal protein 6 homolog",
  "term_label": "centriole replication",
  "gene_symbol": "SASS6"
}